{
  "term_id": "GO:0016477",
  "gene_name": "Cadherin-20",
  "gene": "UniProtKB:Q9HBT6",
  "term_label": "cell migration",
  "gene_symbol": "CDH20"
}